{
  "term_label": "T cell mediated immunity",
  "gene_symbol": "CD8A",
  "gene_name": "T-cell surface glycoprotein CD8 alpha chain",
  "gene": "UniProtKB:P01732",
  "term_id": "GO:0002456"
}